{
  "term_id": "GO:0004115",
  "gene_name": "High affinity cAMP-specific and IBMX-insensitive 3',5'-cyclic phosphodiesterase 8A",
  "gene_symbol": "PDE8A",
  "term_label": "3',5'-cyclic-AMP phosphodiesterase activity",
  "gene": "UniProtKB:O60658"
}